negative regulation of mesenchymal cell apoptotic process involved in metanephric nephron morphogenesis [GO:0072305] (biological process) Relationships: is a type of negative regulation of mesenchymal cell apoptotic process involved in nephron morphogenesis [GO:0072040]; is a type of regulation of mesenchymal cell apoptotic process involved in metanephric nephron morphogenesis [GO:0072304]; is a type of GO:1900212; negatively regulates mesenchymal stem cell maintenance involved in metanephric nephron morphogenesis [GO:0072309]; negatively regulates mesenchymal cell apoptotic process involved in metanephric nephron morphogenesis [GO:1901147] Sources: GOC:mtg_apoptosis, GOC:mtg_kidney_jan10 Definition: Any process that reduces the occurrence or rate of mesenchymal stem cell death by apoptotic process that contributes to the shaping of the nephron in the metanephros. Also known as: negative regulation of mesenchymal stem cell apoptotic process involved in metanephric nephron morphogenesis, negative regulation of mesenchymal stem cell apoptosis involved in metanephric nephron morphogenesis